{
  "term_label": "cell surface receptor protein tyrosine kinase signaling pathway",
  "term_id": "GO:0007169",
  "gene_name": "Sterile alpha motif domain-containing protein 10",
  "gene": "UniProtKB:Q9BYL1",
  "gene_symbol": "SAMD10"
}